{
  "gene": "UniProtKB:Q9BSR8",
  "gene_name": "Protein YIPF4",
  "term_label": "Unknown molecular function",
  "term_id": "UNKNOWN:0001",
  "gene_symbol": "YIPF4"
}